{
  "gene": "UniProtKB:Q9UGJ0",
  "gene_symbol": "PRKAG2",
  "term_label": "protein kinase binding",
  "gene_name": "5'-AMP-activated protein kinase subunit gamma-2",
  "term_id": "GO:0019901"
}